{
  "gene_symbol": "SORBS3",
  "term_id": "GO:0007010",
  "gene": "UniProtKB:O60504",
  "term_label": "cytoskeleton organization",
  "gene_name": "Vinexin"
}